{
  "term_id": "GO:0015629",
  "gene": "UniProtKB:Q16658",
  "gene_name": "Fascin",
  "gene_symbol": "FSCN1",
  "term_label": "actin cytoskeleton"
}